{
  "gene_symbol": "TTI1",
  "gene": "UniProtKB:O43156",
  "term_id": "GO:0005737",
  "term_label": "cytoplasm",
  "gene_name": "TELO2-interacting protein 1 homolog"
}